{
  "gene_symbol": "ECHDC2",
  "gene": "UniProtKB:Q86YB7",
  "gene_name": "Enoyl-CoA hydratase domain-containing protein 2, mitochondrial",
  "term_id": "GO:0005739",
  "term_label": "mitochondrion"
}